pole plasm [GO:0045495] (cellular component) Relationships: is a type of cytoplasm [GO:0005737] Definition: Differentiated cytoplasm associated with a pole (animal, vegetal, anterior, or posterior) of an oocyte, egg or early embryo. References: PMID:17113380 Sources: GOC:kmv Also known as: polar plasm, germ plasm Subtypes: germ plasm [GO:0060293]